{
  "term_label": "negative regulation of BMP signaling pathway",
  "gene_name": "E3 ubiquitin-protein ligase SMURF2",
  "gene_symbol": "SMURF2",
  "gene": "UniProtKB:Q9HAU4",
  "term_id": "GO:0030514"
}